positive regulation of brassinosteroid biosynthetic process [GO:2000488] (BP) Definition: Any process that activates or increases the frequency, rate or extent of brassinosteroid biosynthetic process. Sources: GOC:obol Also known as: positive regulation of brassinosteroid anabolism, positive regulation of brassinosteroid biosynthesis, positive regulation of brassinosteroid formation, positive regulation of brassinosteroid synthesis Relationships: is a type of regulation of brassinosteroid biosynthetic process [GO:0010422]; is a type of positive regulation of steroid biosynthetic process [GO:0010893]; is a type of positive regulation of hormone metabolic process [GO:0032352]; positively regulates brassinosteroid biosynthetic process [GO:0016132]